{
  "term_id": "UNKNOWN:0003",
  "gene_symbol": "PCOLCE2",
  "gene": "UniProtKB:Q9UKZ9",
  "gene_name": "Procollagen C-endopeptidase enhancer 2",
  "term_label": "Unknown cellular component"
}